leading edge cell fate determination [GO:0035028] (biological process) Relationships: is_a cell fate determination [GO:0001709]; is part of leading edge cell fate commitment [GO:0035027] Definition: The process in which a cell becomes capable of differentiating autonomously into a leading edge cell regardless of its environment; upon determination, the cell fate cannot be reversed. Sources: GOC:bf Subtypes: dorsal closure, leading edge cell fate determination [GO:0007393]